{
  "gene": "UniProtKB:Q13237",
  "gene_name": "cGMP-dependent protein kinase 2",
  "term_label": "Unknown molecular function",
  "gene_symbol": "PRKG2",
  "term_id": "UNKNOWN:0001"
}